{
  "gene_name": "Src-like-adapter 2",
  "gene_symbol": "SLA2",
  "gene": "UniProtKB:Q9H6Q3",
  "term_id": "GO:0035591",
  "term_label": "signaling adaptor activity"
}